interleukin-11-mediated signaling pathway [GO:0038154] (biological process) Definition: The series of molecular signals initiated by the binding of interleukin-11 to its receptor on the surface of a target cell, and ending with the regulation of a downstream cellular process, e.g. transcription. Also known as: IL-11-mediated signaling pathway, interleukin-11-mediated signalling pathway Relationships: is a type of cytokine-mediated signaling pathway [GO:0019221] Sources: GOC:nhn, GOC:signaling